{
  "gene_name": "FHF complex subunit HOOK-interacting protein 2B",
  "gene_symbol": "FHIP2B",
  "term_label": "Unknown molecular function",
  "term_id": "UNKNOWN:0001",
  "gene": "UniProtKB:Q86V87"
}